larval locomotory behavior [GO:0008345] (biological process) Subtypes: larval walking behavior [GO:0008346], larval wandering behavior [GO:0035180], larval burrowing behavior [GO:0035181] Sources: GOC:ai Also known as: larval locomotory behaviour Note: See also the biological process term 'locomotory behavior ; GO:0007626'. Relationships: is_a GO:0007626; is a type of larval behavior [GO:0030537] Definition: Locomotory behavior in a larval (immature) organism.